{
  "term_label": "plasma membrane",
  "gene_symbol": "PCDHB13",
  "term_id": "GO:0005886",
  "gene": "UniProtKB:Q9Y5F0",
  "gene_name": "Protocadherin beta-13"
}